{
  "gene_symbol": "OPN1MW3",
  "term_label": "photoreceptor outer segment",
  "gene_name": "Medium-wave-sensitive opsin 3",
  "term_id": "GO:0001750",
  "gene": "UniProtKB:P0DN78"
}